regulation of cellular response to hepatocyte growth factor stimulus [GO:2001112] (biological process) Sources: GOC:obol Definition: Any process that modulates the frequency, rate or extent of cellular response to hepatocyte growth factor stimulus. Subtypes: negative regulation of cellular response to hepatocyte growth factor stimulus [GO:2001113], GO:2001114 Relationships: is a type of GO:0090287; regulates cellular response to hepatocyte growth factor stimulus [GO:0035729] Also known as: regulation of cellular response to HGF stimulus